{
  "gene_name": "SH3 domain-containing YSC84-like protein 1",
  "gene_symbol": "SH3YL1",
  "term_label": "ruffle membrane",
  "gene": "UniProtKB:Q96HL8",
  "term_id": "GO:0032587"
}